UAA codon-amino acid adaptor activity [GO:0033411] (molecular function) Definition: A triplet codon-amino acid adaptor activity that recognizes a UAA codon. Sources: GOC:mah Also known as: TAA codon-amino acid adaptor activity Note: Note that in the standard genetic code, TAA is a stop codon (ochre) and is not normally read by a tRNA. Relationships: is a type of GO:0030533